{
  "gene": "UniProtKB:P32298",
  "term_id": "GO:0004672",
  "term_label": "protein kinase activity",
  "gene_name": "G protein-coupled receptor kinase 4",
  "gene_symbol": "GRK4"
}